{
  "term_label": "transmembrane transport",
  "term_id": "GO:0055085",
  "gene_symbol": "SLC2A6",
  "gene": "UniProtKB:Q9UGQ3",
  "gene_name": "Solute carrier family 2, facilitated glucose transporter member 6"
}